{
  "gene_name": "Megakaryocyte and platelet inhibitory receptor G6b",
  "term_id": "GO:0035855",
  "term_label": "megakaryocyte development",
  "gene": "UniProtKB:O95866",
  "gene_symbol": "MPIG6B"
}